{
  "gene": "UniProtKB:Q9H7X7",
  "gene_symbol": "IFT22",
  "gene_name": "Intraflagellar transport protein 22 homolog",
  "term_id": "GO:0012505",
  "term_label": "endomembrane system"
}